ubiquitin ligase complex [GO:0000151] (cellular component) Relationships: is a type of intracellular protein-containing complex [GO:0140535]; is a type of transferase complex [GO:1990234] Definition: A protein complex that includes a ubiquitin-protein ligase and enables ubiquitin protein ligase activity. The complex also contains other proteins that may confer substrate specificity on the complex. References: PMID:9529603 Sources: GOC:jh2 Subtypes: GO:0000152, cytoplasmic ubiquitin ligase complex [GO:0000153], cullin-RING ubiquitin ligase complex [GO:0031461], HULC complex [GO:0033503], GID complex [GO:0034657], Dsc E3 ubiquitin ligase complex [GO:0044695], LUBAC complex [GO:0071797], Rad6-Rad18 complex [GO:0097505], GO:1990352, Fused-Smurf ubiquitin ligase complex [GO:1990353], Parkin-FBXW7-Cul1 ubiquitin ligase complex [GO:1990452]